{
  "gene": "UniProtKB:Q9GZZ6",
  "gene_symbol": "CHRNA10",
  "term_label": "transmembrane transporter complex",
  "gene_name": "Neuronal acetylcholine receptor subunit alpha-10",
  "term_id": "GO:1902495"
}